immunoglobulin production in mucosal tissue [GO:0002426] (biological process) Sources: GOC:jal Also known as: antibody production in mucosal tissue Definition: The synthesis and release of immunoglobulin in the mucosal tissue. Note: Note that this term is in the subset of terms that should not be used for direct gene product annotation. Instead, select one of the 'regulation' children terms. Relationships: is_a GO:0002381; is part of mucosal immune response [GO:0002385] Regulation: RO_0002211 by regulation of immunoglobulin production in mucosal tissue [GO:2000557]; positively regulated by positive regulation of immunoglobulin production in mucosal tissue [GO:2000558]